{
  "term_id": "GO:0042806",
  "gene_symbol": "CLEC17A",
  "gene": "UniProtKB:Q6ZS10",
  "term_label": "fucose binding",
  "gene_name": "C-type lectin domain family 17, member A"
}